{
  "term_id": "GO:0015020",
  "gene_symbol": "UGT2A2",
  "term_label": "glucuronosyltransferase activity",
  "gene_name": "UDP-glucuronosyltransferase 2A2",
  "gene": "UniProtKB:P0DTE5"
}